sequence-specific double-stranded DNA binding [GO:1990837] (molecular function) Also known as: sequence-specific dsDNA binding Sources: GOC:dos, GOC:sl Relationships: is a type of double-stranded DNA binding [GO:0003690]; is a type of sequence-specific DNA binding [GO:0043565] Subtypes: GO:0000182, transcription cis-regulatory region binding [GO:0000976], DNA replication origin binding [GO:0003688], GO:0003693, satellite DNA binding [GO:0003696], GO:0019237, GO:0031634, GO:0044374, tDNA binding [GO:0071443], GO:0141180, piRNA cluster binding [GO:1990470] Definition: Binding to double-stranded DNA of a specific nucleotide composition, e.g. GC-rich DNA binding, or with a specific sequence motif or type of DNA, e.g. promotor binding or rDNA binding.